paranodal junction [GO:0033010] (cellular component) Also known as: axoglial septate junction, paranodal axoglial junction, paranodal septate junction Definition: A highly specialized cell-cell junction found in vertebrates, which forms between a neuron and a glial cell, and has structural similarity to Drosophila septate junctions. It flanks the node of Ranvier in myelinated nerve and electrically isolates the myelinated from unmyelinated nerve segments and physically separates the voltage-gated sodium channels at the node from the cluster of potassium channels underneath the myelin sheath. References: PMID:11395001, PMID:14630217 Relationships: is a type of GO:0005911